{
  "gene_name": "Proliferation-associated protein 2G4",
  "term_id": "UNKNOWN:0003",
  "gene_symbol": "PA2G4",
  "gene": "UniProtKB:Q9UQ80",
  "term_label": "Unknown cellular component"
}